{
  "term_label": "RNA polymerase II cis-regulatory region sequence-specific DNA binding",
  "gene_name": "Paired box protein Pax-8",
  "gene_symbol": "PAX8",
  "term_id": "GO:0000978",
  "gene": "UniProtKB:Q06710"
}